positive regulation of Notch signaling pathway [GO:0045747] (biological process) Definition: Any process that activates or increases the frequency, rate or extent of the Notch signaling pathway. Sources: GOC:go_curators Also known as: positive regulation of N signaling pathway, positive regulation of N signalling pathway, positive regulation of Notch signalling pathway, up regulation of Notch signaling pathway, up-regulation of Notch signaling pathway, upregulation of Notch signaling pathway, activation of Notch signaling pathway, stimulation of Notch signaling pathway Relationships: is_a regulation of Notch signaling pathway [GO:0008593]; is a type of positive regulation of signal transduction [GO:0009967]; positively regulates Notch signaling pathway [GO:0007219]